{
  "term_label": "phospholipid scramblase activity",
  "gene": "UniProtKB:Q4KMQ2",
  "gene_symbol": "ANO6",
  "term_id": "GO:0017128",
  "gene_name": "Anoctamin-6"
}